{
  "term_id": "UNKNOWN:0001",
  "gene": "UniProtKB:Q9ULQ1",
  "gene_symbol": "TPCN1",
  "gene_name": "Two pore channel protein 1",
  "term_label": "Unknown molecular function"
}